{
  "gene": "UniProtKB:Q9BZE9",
  "term_label": "glucose homeostasis",
  "gene_symbol": "ASPSCR1",
  "term_id": "GO:0042593",
  "gene_name": "Tether containing UBX domain for GLUT4"
}